{
  "gene_name": "LanC-like protein 2",
  "term_id": "GO:0005634",
  "gene_symbol": "LANCL2",
  "term_label": "nucleus",
  "gene": "UniProtKB:Q9NS86"
}